{
  "gene_symbol": "RAB31",
  "term_id": "GO:0006886",
  "term_label": "intracellular protein transport",
  "gene_name": "Ras-related protein Rab-31",
  "gene": "UniProtKB:Q13636"
}